{
  "gene": "UniProtKB:P56539",
  "gene_name": "Caveolin-3",
  "term_label": "regulation of membrane potential",
  "gene_symbol": "CAV3",
  "term_id": "GO:0042391"
}